{
  "term_label": "tolerance induction to self antigen",
  "gene_name": "Tyrosine-protein kinase Lyn",
  "term_id": "GO:0002513",
  "gene_symbol": "LYN",
  "gene": "UniProtKB:P07948"
}